{
  "gene_symbol": "EOMES",
  "term_id": "GO:0005634",
  "gene": "UniProtKB:O95936",
  "term_label": "nucleus",
  "gene_name": "Eomesodermin homolog"
}